{
  "gene": "UniProtKB:Q15435",
  "term_label": "protein phosphatase regulator activity",
  "term_id": "GO:0019888",
  "gene_symbol": "PPP1R7",
  "gene_name": "Protein phosphatase 1 regulatory subunit 7"
}